{
  "term_label": "cell-cell adhesion",
  "gene": "UniProtKB:Q92823",
  "term_id": "GO:0098609",
  "gene_name": "Neuronal cell adhesion molecule",
  "gene_symbol": "NRCAM"
}